2,4-dichlorophenoxyacetic acid catabolic process [GO:0046300] (biological process) Also known as: 2,4-dichlorophenoxyacetic acid breakdown, 2,4-dichlorophenoxyacetic acid catabolism, 2,4-dichlorophenoxyacetic acid degradation Definition: The chemical reactions and pathways resulting in the breakdown of 2,4-dichlorophenoxyacetic acid, a chlorinated phenoxy compound which functions as a systemic herbicide and is used to control many types of broadleaf weeds. Relationships: is a type of GO:0018901; is_a monocarboxylic acid catabolic process [GO:0072329]; is a type of ether catabolic process [GO:1901502] Sources: GOC:ai, UM-BBD_pathwayID:2,4-d